{
  "term_id": "GO:0005829",
  "term_label": "cytosol",
  "gene_name": "Ubiquitin carboxyl-terminal hydrolase 13",
  "gene_symbol": "USP13",
  "gene": "UniProtKB:Q92995"
}